{
  "term_label": "ubiquitin-protein transferase activity",
  "gene_symbol": "MYLIP",
  "term_id": "GO:0004842",
  "gene": "UniProtKB:Q8WY64",
  "gene_name": "E3 ubiquitin-protein ligase MYLIP"
}